{
  "gene_symbol": "RFC5",
  "gene": "UniProtKB:P40937",
  "term_label": "DNA replication factor C complex",
  "gene_name": "Replication factor C subunit 5",
  "term_id": "GO:0005663"
}